{
  "gene_symbol": "RPGRIP1L",
  "gene": "UniProtKB:Q68CZ1",
  "term_label": "thromboxane A2 receptor binding",
  "term_id": "GO:0031870",
  "gene_name": "Protein fantom"
}